{
  "gene_symbol": "IQCB1",
  "term_label": "Unknown molecular function",
  "gene": "UniProtKB:Q15051",
  "term_id": "UNKNOWN:0001",
  "gene_name": "IQ calmodulin-binding motif-containing protein 1"
}